methylosome [GO:0034709] (cellular component) Also known as: 20S methylosome, 20S methyltransferase complex References: PMID:11713266, PMID:11756452 Relationships: is a type of methyltransferase complex [GO:0034708]; is part of cytoplasm [GO:0005737] Definition: A large (20 S) protein complex that possesses protein arginine methyltransferase activity and modifies specific arginines to dimethylarginines in the arginine- and glycine-rich domains of several spliceosomal Sm proteins, thereby targeting these proteins to the survival of motor neurons (SMN) complex for assembly into small nuclear ribonucleoprotein (snRNP) core particles. Proteins found in the methylosome include the methyltransferase JBP1 (PRMT5), pICln (CLNS1A), MEP50 (WDR77), and unmethylated forms of SM proteins that have RG domains.